{
  "gene_symbol": "TENM2",
  "gene_name": "Teneurin-2",
  "term_label": "neuron development",
  "gene": "UniProtKB:Q9NT68",
  "term_id": "GO:0048666"
}